{
  "gene_symbol": "KRTAP2-3",
  "gene_name": "Keratin-associated protein 2-3",
  "term_label": "Unknown biological process",
  "gene": "UniProtKB:P0C7H8",
  "term_id": "UNKNOWN:0002"
}